snRNA import into nucleus [GO:0061015] (biological process) Sources: GOC:ascb_2009, GOC:dph, GOC:tb Definition: The directed movement of snRNA, small nuclear ribonucleic acid into the nucleus. Relationships: is a type of GO:0006404; is a type of snRNA transport [GO:0051030]